{
  "gene_name": "C2 domain-containing protein 5",
  "gene": "UniProtKB:Q86YS7",
  "term_label": "positive regulation of vesicle fusion",
  "gene_symbol": "C2CD5",
  "term_id": "GO:0031340"
}